{
  "gene": "UniProtKB:Q13153",
  "gene_symbol": "PAK1",
  "gene_name": "Serine_threonine-protein kinase PAK 1",
  "term_label": "regulation of MAPK cascade",
  "term_id": "GO:0043408"
}